positive regulation of signal transduction involved in conjugation with cellular fusion [GO:0060239] (biological process) Definition: Any process that increases the rate, frequency or extent of signal transduction involved in conjugation with cellular fusion. Relationships: is_a positive regulation of signal transduction [GO:0009967]; is a type of positive regulation of conjugation with cellular fusion [GO:0031139]; is a type of regulation of signal transduction involved in conjugation with cellular fusion [GO:0060238]; positively regulates signal transduction involved in positive regulation of conjugation with cellular fusion [GO:0032005] Sources: GOC:dph, GOC:tb Subtypes: positive regulation of pheromone-dependent signal transduction involved in conjugation with cellular fusion [GO:0090028]